{
  "gene_symbol": "UCK2",
  "term_label": "uridine kinase activity",
  "term_id": "GO:0004849",
  "gene_name": "Uridine-cytidine kinase 2",
  "gene": "UniProtKB:Q9BZX2"
}